{
  "term_label": "7SK snRNA binding",
  "gene_name": "Protein HEXIM2",
  "term_id": "GO:0097322",
  "gene": "UniProtKB:Q96MH2",
  "gene_symbol": "HEXIM2"
}